{
  "gene_symbol": "CALM3",
  "term_label": "centrosome",
  "gene": "UniProtKB:P0DP25",
  "gene_name": "Calmodulin-3",
  "term_id": "GO:0005813"
}